{
  "gene_symbol": "RAB2A",
  "gene": "UniProtKB:P61019",
  "gene_name": "Ras-related protein Rab-2A",
  "term_id": "GO:0000139",
  "term_label": "Golgi membrane"
}